{
  "term_id": "GO:0038127",
  "term_label": "ERBB signaling pathway",
  "gene": "UniProtKB:Q06124",
  "gene_symbol": "PTPN11",
  "gene_name": "Tyrosine-protein phosphatase non-receptor type 11"
}